cingulate gyrus development [GO:0021765] (biological process) Definition: The progression of the cingulate gyrus over time from its initial formation until its mature state. The cingulate gyrus is a ridge in the cerebral cortex located dorsal to the corpus callosum. Sources: GOC:cls, GOC:dgh, GOC:dph, GOC:jid, GO_REF:0000021 Relationships: is a type of anatomical structure development [GO:0048856]; is part of limbic system development [GO:0021761]